{
  "term_label": "molecular adaptor activity",
  "gene_name": "Pericentriolar material 1 protein",
  "gene": "UniProtKB:Q15154",
  "gene_symbol": "PCM1",
  "term_id": "GO:0060090"
}